positive regulation of anthocyanin metabolic process [GO:0031539] (biological process) Definition: Any process that activates or increases the frequency, rate or extent of chemical reactions and pathways involving anthocyanins. Relationships: is a type of GO:0009893; is a type of regulation of anthocyanin metabolic process [GO:0031537]; positively regulates anthocyanin-containing compound metabolic process [GO:0046283] Subtypes: GO:0031542, positive regulation of anthocyanin catabolic process [GO:1900002] Sources: GOC:mah Also known as: positive regulation of anthocyanin metabolism, up regulation of anthocyanin metabolic process, up-regulation of anthocyanin metabolic process, upregulation of anthocyanin metabolic process, activation of anthocyanin metabolic process, stimulation of anthocyanin metabolic process